U6 snRNP [GO:0005688] (CC) Also known as: snRNP U6 Definition: A ribonucleoprotein complex that contains small nuclear RNA U6, the Lsm2-8 heptameric ring complex, as well as several proteins that are unique to the U6 snRNP, most of which remain associated with the U6 snRNA both while the U6 snRNP is free or assembled into the U4/U6 snRNP or into a series of spliceosomal complexes. Sources: GOC:krc, GOC:mah, ISBN:0879695897 Relationships: is_a spliceosomal snRNP complex [GO:0097525]; has part Lsm2-8 complex [GO:0120115]